{
  "gene_symbol": "NES",
  "term_label": "CCR5 chemokine receptor binding",
  "term_id": "GO:0031730",
  "gene_name": "Nestin",
  "gene": "UniProtKB:P48681"
}